symbiont-mediated suppression of cytoplasmic pattern recognition receptor signaling pathway [GO:0039537] (biological process) Note: Note that this term should be used when the symbiont directly inhibits a component of a host cytoplasmic receptor signaling pathway. In cases where the symbiont modifies its own molecules (proteins, DNA, RNA, lipids) to avoid recognition by the host, consider annotating to evasion of symbiont recognition by host pattern recognition receptor ; GO:0141141. Subtypes: symbiont-mediated suppression of host cytoplasmic pattern recognition receptor signaling pathway via inhibition of RIG-I activity [GO:0039540], symbiont-mediated suppression of host cytoplasmic pattern recognition receptor signaling pathway via inhibition of MAVS activity [GO:0039545], symbiont-mediated suppression of host cytoplasmic pattern recognition receptor signaling pathway via inhibition of IRF3 activity [GO:0039548], symbiont-mediated suppression of host cytoplasmic pattern recognition receptor signaling pathway via inhibition of MDA-5 activity [GO:0039554], symbiont-mediated suppression of host cytoplasmic pattern recognition receptor signaling pathway via inhibition of IRF7 activity [GO:0039557], GO:0039723, symbiont-mediated suppression of host cytoplasmic pattern recognition receptor signaling pathway via inhibition of IKBKE activity [GO:0039724], symbiont-mediated suppression of host cGAS-STING signal transduction [GO:0141074], symbiont-mediated suppression of host inflammasome-mediated signal transduction [GO:0141081] Sources: GOC:bf, GOC:jl Also known as: suppression by virus of host cytoplasmic pattern recognition receptor signaling pathway in response to virus, suppression by virus of host viral-induced cytoplasmic pattern recognition receptor signalling pathway, suppression by virus of host viral-induced cytoplasmic pattern recognition receptor signaling pathway, suppression by virus of host RIG-I-like receptor (RLR) signaling pathway, suppression by virus of host RIG-I/MDA5 signaling pathway, suppression by virus of host RIG-like helicase signaling pathway, suppression by virus of host RIG-like receptor signaling pathway, suppression by virus of host RLR signaling pathway Definition: A process in which a symbiont interferes with, inhibits or disrupts a cytoplasmic pattern recognition receptor signaling pathway. This is a mechanism by which the virus evades the host innate immune response. Relationships: is a type of symbiont-mediated suppression of host pathogen-associated molecular pattern receptor signaling pathway [GO:0052078]